atrioventricular valve morphogenesis [GO:0003181] (biological process) Subtypes: GO:0003183, tricuspid valve morphogenesis [GO:0003186] Also known as: AV valve morphogenesis Relationships: is a type of heart valve morphogenesis [GO:0003179]; is part of atrioventricular valve development [GO:0003171] Sources: GOC:mtg_heart Definition: The process in which the structure of the atrioventricular valve is generated and organized.